{
  "gene": "UniProtKB:Q9HCG8",
  "term_label": "RNA binding",
  "gene_name": "Pre-mRNA-splicing factor CWC22 homolog",
  "term_id": "GO:0003723",
  "gene_symbol": "CWC22"
}